symbiont-mediated disruption of host cell wall [GO:0052009] (biological process) Also known as: disassembly by symbiont of host cell wall, disruption by symbiont of host cell wall Subtypes: symbiont entry into host cell via disruption of host cell wall peptidoglycan [GO:0098932], symbiont entry into host cell via disruption of host cell envelope lipopolysaccharide [GO:0098995] Sources: ISBN:0198547684 Definition: The process in which an organism effects a change that impairs the structure or function of the host cell wall. The host is defined as the larger of the organisms involved in a symbiotic interaction. Relationships: is a type of symbiont-mediated disruption of host cell envelope [GO:0098933]